{
  "gene": "UniProtKB:Q13185",
  "term_id": "GO:0031507",
  "term_label": "heterochromatin formation",
  "gene_symbol": "CBX3",
  "gene_name": "Chromobox protein homolog 3"
}